stizolobate synthase activity [GO:0050297] (molecular function) Sources: RHEA:21220 Also known as: DOPA dioxygenase activity, 3,4-dihydroxy-L-phenylalanine:oxygen 4,5-oxidoreductase (recyclizing) Relationships: is a type of GO:0016702 Definition: Catalysis of the reaction: L-dopa + O2 = 4-(L-alanin-3-yl)-2-hydroxy-cis,cis-muconate 6-semialdehyde + H+.